{
  "term_label": "DNA-binding transcription factor activity, RNA polymerase II-specific",
  "gene_name": "Heart- and neural crest derivatives-expressed protein 1",
  "term_id": "GO:0000981",
  "gene": "UniProtKB:O96004",
  "gene_symbol": "HAND1"
}